detection of pheromone [GO:0043695] (BP) Relationships: is a type of detection of chemical stimulus [GO:0009593]; is a type of response to pheromone [GO:0019236] Definition: The series of events in which a pheromone stimulus is received by a cell and converted into a molecular signal. Sources: GOC:mah